{
  "gene_symbol": "ANKRD7",
  "term_label": "Unknown cellular component",
  "gene": "UniProtKB:Q92527",
  "gene_name": "Ankyrin repeat domain-containing protein 7",
  "term_id": "UNKNOWN:0003"
}